{
  "gene_name": "DNA ligase 4",
  "term_label": "nucleotide-excision repair, DNA gap filling",
  "term_id": "GO:0006297",
  "gene": "UniProtKB:P49917",
  "gene_symbol": "LIG4"
}